{
  "term_id": "GO:0006357",
  "gene": "UniProtKB:Q13888",
  "gene_name": "General transcription factor IIH subunit 2",
  "term_label": "regulation of transcription by RNA polymerase II",
  "gene_symbol": "GTF2H2"
}